negative regulation of translation in response to osmotic stress [GO:0032061] (biological process) Relationships: is a type of GO:0032055; is a type of GO:0043557 Sources: GOC:mah Definition: Any process that stops, prevents or reduces the rate of translation as a result of a stimulus indicating an increase or decrease in the concentration of solutes outside the organism or cell. Also known as: down regulation of translation in response to osmotic stress, down-regulation of translation in response to osmotic stress, downregulation of translation in response to osmotic stress, inhibition of translation in response to osmotic stress Subtypes: negative regulation of translational initiation in response to osmotic stress [GO:0032063]